{
  "term_id": "GO:0120013",
  "gene_symbol": "TTPA",
  "term_label": "lipid transfer activity",
  "gene": "UniProtKB:P49638",
  "gene_name": "Alpha-tocopherol transfer protein"
}